{
  "gene": "UniProtKB:Q9UKG1",
  "term_id": "GO:0043422",
  "gene_symbol": "APPL1",
  "gene_name": "DCC-interacting protein 13-alpha",
  "term_label": "protein kinase B binding"
}